{
  "gene": "UniProtKB:P58181",
  "term_label": "plasma membrane",
  "term_id": "GO:0005886",
  "gene_name": "Olfactory receptor 10A3",
  "gene_symbol": "OR10A3"
}